myo-inositol hexakisphosphate biosynthetic process [GO:0010264] (biological process) Definition: The chemical reactions and pathways resulting in the formation of phytic acid, myo-inositol hexakisphosphate, a regulator of intracellular signaling, a highly abundant animal anti-nutrient and a phosphate and mineral storage compound in plant seeds. Also known as: myo-inositol hexakisphosphate anabolism, myo-inositol hexakisphosphate biosynthesis, myo-inositol hexakisphosphate formation, myo-inositol hexakisphosphate synthesis, phytate biosynthesis, phytate biosynthetic process Relationships: is a type of inositol phosphate biosynthetic process [GO:0032958] Subtypes: myo-inositol hexakisphosphate biosynthetic process, lipid-dependent [GO:0033545], myo-inositol hexakisphosphate biosynthetic process, lipid-independent [GO:0033548] References: PMID:16107538